{
  "term_label": "cytoplasm",
  "term_id": "GO:0005737",
  "gene_symbol": "TRIM48",
  "gene": "UniProtKB:Q8IWZ4",
  "gene_name": "E3 ubiquitin-protein ligase TRIM48"
}